{
  "gene": "UniProtKB:Q13724",
  "term_id": "GO:0006487",
  "term_label": "protein N-linked glycosylation",
  "gene_name": "Mannosyl-oligosaccharide glucosidase",
  "gene_symbol": "MOGS"
}